negative regulation of interleukin-12 production [GO:0032695] (biological process) Definition: Any process that stops, prevents, or reduces the frequency, rate, or extent of interleukin-12 production. Relationships: is a type of negative regulation of cytokine production [GO:0001818]; is a type of GO:0032655; negatively regulates GO:0032615 Also known as: down regulation of interleukin-12 production, down-regulation of interleukin-12 production, downregulation of interleukin-12 production, negative regulation of IL-12 production, inhibition of interleukin-12 production, negative regulation of interleukin-12 biosynthetic process, negative regulation of interleukin-12 secretion, negative regulation of CLMF production, negative regulation of NKSF production Sources: GOC:mah